{
  "gene_name": "Hyaluronidase PH-20",
  "term_id": "GO:0004415",
  "term_label": "hyalurononglucosaminidase activity",
  "gene": "UniProtKB:P38567",
  "gene_symbol": "SPAM1"
}